lipid modification [GO:0030258] (biological process) Relationships: is a type of GO:0006629 Sources: GOC:mah Definition: The covalent alteration of one or more fatty acids in a lipid, resulting in a change in the properties of the lipid. Subtypes: lipid hydroxylation [GO:0002933], lipid oxidation [GO:0034440], GO:0046834, phospholipid dephosphorylation [GO:0046839], GO:0120322